{
  "term_id": "GO:0030198",
  "term_label": "extracellular matrix organization",
  "gene": "UniProtKB:Q14993",
  "gene_symbol": "COL19A1",
  "gene_name": "Collagen alpha-1(XIX) chain"
}